regulation of lysosome size [GO:0062196] (biological process) Definition: Any process that modulates the size of a lysosome. Relationships: is a type of regulation of cellular component size [GO:0032535] References: PMID:31314175